positive regulation of monocyte antigen processing and presentation [GO:0002615] (biological process) Definition: Any process that activates or increases the frequency, rate, or extent of monocyte antigen processing and presentation. Sources: GOC:add Also known as: up regulation of monocyte antigen processing and presentation, up-regulation of monocyte antigen processing and presentation, upregulation of monocyte antigen processing and presentation, activation of monocyte antigen processing and presentation, stimulation of monocyte antigen processing and presentation Relationships: is_a positive regulation of antigen processing and presentation [GO:0002579]; is a type of regulation of monocyte antigen processing and presentation [GO:0002613]; positively regulates monocyte antigen processing and presentation [GO:0002471]